{
  "term_label": "Unknown molecular function",
  "gene_symbol": "TRAPPC6A",
  "gene_name": "Trafficking protein particle complex subunit 6A",
  "term_id": "UNKNOWN:0001",
  "gene": "UniProtKB:O75865"
}